protein antigen binding [GO:1990405] (molecular function) References: PMID:9360996 Definition: Binding to a protein antigen. Relationships: is_a antigen binding [GO:0003823]; is a type of protein binding [GO:0005515]